neutrophil activation involved in immune response [GO:0002283] (biological process) Sources: GOC:add, ISBN:0781735149 Relationships: is a type of myeloid cell activation involved in immune response [GO:0002275]; is a type of GO:0042119 Also known as: neutrophil activation during immune response Definition: The change in morphology and behavior of a neutrophil resulting from exposure to a cytokine, chemokine, cellular ligand, or soluble factor, leading to the initiation or perpetuation of an immune response.